tatiopterin metabolic process [GO:1900869] (biological process) Sources: GOC:TermGenie, GOC:mengo_curators Also known as: tatiopterin metabolism Definition: The chemical reactions and pathways involving tatiopterin. Relationships: is_a phosphorus metabolic process [GO:0006793]; is a type of carboxylic acid metabolic process [GO:0019752]; is a type of pteridine-containing compound metabolic process [GO:0042558] Subtypes: GO:1900870